{
  "term_id": "GO:0003777",
  "gene_symbol": "KIF23",
  "gene": "UniProtKB:Q02241",
  "term_label": "microtubule motor activity",
  "gene_name": "Kinesin-like protein KIF23"
}